negative regulation of myoblast differentiation [GO:0045662] (biological process) Sources: CL:0000056, GOC:go_curators, GOC:mtg_muscle Relationships: is a type of negative regulation of cell differentiation [GO:0045596]; is_a regulation of myoblast differentiation [GO:0045661]; negatively regulates myoblast differentiation [GO:0045445] Definition: Any process that stops, prevents, or reduces the frequency, rate or extent of myoblast differentiation. A myoblast is a mononucleate cell type that, by fusion with other myoblasts, gives rise to the myotubes that eventually develop into skeletal muscle fibers. Subtypes: negative regulation of cardiac muscle cell myoblast differentiation [GO:2000691] Also known as: down regulation of myoblast differentiation, down-regulation of myoblast differentiation, downregulation of myoblast differentiation, inhibition of myoblast differentiation